scyllo-inositol dehydrogenase (NADP+) activity [GO:0102497] (molecular function) Sources: EC:1.1.1.371, GOC:pz Definition: Catalysis of the reaction: scyllo-inositol + NADP = 2,4,6/3,5-pentahydroxycyclohexanone + NADPH + H+. Relationships: is a type of oxidoreductase activity, acting on the CH-OH group of donors, NAD or NADP as acceptor [GO:0016616]